{
  "gene_symbol": "TIMP4",
  "term_label": "extracellular space",
  "gene_name": "Metalloproteinase inhibitor 4",
  "term_id": "GO:0005615",
  "gene": "UniProtKB:Q99727"
}